{
  "gene": "UniProtKB:Q16566",
  "term_label": "calcium-dependent protein serine/threonine kinase activity",
  "gene_symbol": "CAMK4",
  "term_id": "GO:0009931",
  "gene_name": "Calcium_calmodulin-dependent protein kinase type IV"
}